{
  "gene_symbol": "PTH",
  "gene_name": "Parathyroid hormone",
  "gene": "UniProtKB:P01270",
  "term_label": "hormone activity",
  "term_id": "GO:0005179"
}